negative regulation of protein-containing complex assembly [GO:0031333] (biological process) Relationships: is a type of regulation of protein-containing complex assembly [GO:0043254]; is a type of GO:0051129; negatively regulates protein-containing complex assembly [GO:0065003] Also known as: down regulation of protein complex assembly, down-regulation of protein complex assembly, downregulation of protein complex assembly, inhibition of protein complex assembly, negative regulation of protein complex assembly Definition: Any process that stops, prevents, or reduces the frequency, rate or extent of protein complex assembly. Subtypes: negative regulation of exocyst assembly [GO:0001929], negative regulation of synaptic vesicle priming [GO:0010809], negative regulation of RNA polymerase II transcription preinitiation complex assembly [GO:0017055], negative regulation of protein polymerization [GO:0032272], negative regulation of protein oligomerization [GO:0032460], negative regulation of integrin activation [GO:0033624], negative regulation of SNARE complex assembly [GO:0035544], negative regulation of pseudohyphal septin ring assembly [GO:0062166], GO:0071802, negative regulation of AIM2 inflammasome complex assembly [GO:0140972], negative regulation of non-canonical inflammasome complex assembly [GO:0160076], negative regulation of nodal receptor complex assembly [GO:1900124], negative regulation of NLRP3 inflammasome complex assembly [GO:1900226], negative regulation of starch utilization system complex assembly [GO:1900513], negative regulation of formation of translation initiation ternary complex [GO:1901191], GO:1901194, negative regulation of ripoptosome assembly involved in necroptotic process [GO:1902443], negative regulation of death-inducing signaling complex assembly [GO:1903073], negative regulation of DNA recombinase mediator complex assembly [GO:1903873], negative regulation of VCP-NPL4-UFD1 AAA ATPase complex assembly [GO:1904240], negative regulation of Wnt-Frizzled-LRP5/6 complex assembly [GO:1904723], negative regulation of shelterin complex assembly [GO:1904791], negative regulation of beta-catenin-TCF complex assembly [GO:1904864], negative regulation of telomerase catalytic core complex assembly [GO:1904883], negative regulation of apoptosome assembly [GO:1905101], GO:1905444, negative regulation of myosin II filament assembly [GO:1905510], GO:1905536, negative regulation of kinetochore assembly [GO:1905560], negative regulation of FACT complex assembly [GO:1905645], negative regulation of Atg1/ULK1 kinase complex assembly [GO:1905865], negative regulation of mediator complex assembly [GO:2001177] Sources: GOC:mah